{
  "term_label": "positive regulation of neuron projection development",
  "gene_name": "Twinfilin-2",
  "gene_symbol": "TWF2",
  "term_id": "GO:0010976",
  "gene": "UniProtKB:Q6IBS0"
}